negative regulation of protein oligomerization [GO:0032460] (biological process) Also known as: down regulation of protein oligomerization, down-regulation of protein oligomerization, downregulation of protein oligomerization, inhibition of protein oligomerization Definition: Any process that stops, prevents, or reduces the frequency, rate or extent of protein oligomerization. Relationships: is a type of negative regulation of protein-containing complex assembly [GO:0031333]; is a type of GO:0032459; negatively regulates protein complex oligomerization [GO:0051259] Sources: GOC:mah Subtypes: GO:0032463, negative regulation of protein tetramerization [GO:1901091]